{
  "gene_symbol": "UTP4",
  "term_label": "regulation of DNA-templated transcription",
  "gene_name": "U3 small nucleolar RNA-associated protein 4 homolog",
  "gene": "UniProtKB:Q969X6",
  "term_id": "GO:0006355"
}